{
  "gene": "UniProtKB:Q9BTA9",
  "term_label": "RNA polymerase II complex binding",
  "term_id": "GO:0000993",
  "gene_name": "WW domain-containing adapter protein with coiled-coil",
  "gene_symbol": "WAC"
}